{
  "gene": "UniProtKB:Q15459",
  "gene_symbol": "SF3A1",
  "gene_name": "Splicing factor 3A subunit 1",
  "term_id": "UNKNOWN:0002",
  "term_label": "Unknown biological process"
}